regulation of the force of skeletal muscle contraction [GO:0014728] (biological process) Sources: GOC:mtg_muscle Definition: Any process that modulates the frequency, rate or extent of the force of skeletal muscle contraction. The force of skeletal muscle contraction is produced by acto-myosin interaction processes through the formation of cross bridges. Relationships: is a type of regulation of skeletal muscle contraction by chemo-mechanical energy conversion [GO:0014862]